chloroplast-nucleus signaling pathway [GO:0010019] (BP) Also known as: chloroplast-nucleus signalling pathway Relationships: is a type of intracellular signal transduction [GO:0035556] Definition: The process in which a molecular signal is transduced between the chloroplast and nucleus, such that expression of nuclear encoding photosynthetic proteins is coupled with chloroplast biogenesis. References: PMID:8972595